{
  "term_id": "UNKNOWN:0001",
  "gene_name": "Ribosomal protein S6 kinase delta-1",
  "gene": "UniProtKB:Q96S38",
  "term_label": "Unknown molecular function",
  "gene_symbol": "RPS6KC1"
}